vesicle-mediated transport to the plasma membrane [GO:0098876] (biological process) Relationships: is a type of GO:0016192; is a type of localization within membrane [GO:0051668]; has part GO:0006887 Subtypes: GO:0006893, endocytic recycling [GO:0032456], neurotransmitter receptor transport to plasma membrane [GO:0098877] Sources: GOC:dos Definition: The directed movement of substances to the plasma membrane in transport vesicles that fuse with the plasma membrane by exocytosis.